{
  "term_label": "guanyl-nucleotide exchange factor activity",
  "gene_symbol": "ARHGEF28",
  "gene_name": "Rho guanine nucleotide exchange factor 28",
  "term_id": "GO:0005085",
  "gene": "UniProtKB:Q8N1W1"
}